{
  "gene_name": "Synaptosomal-associated protein 25",
  "gene": "UniProtKB:P60880",
  "term_id": "GO:0005886",
  "term_label": "plasma membrane",
  "gene_symbol": "SNAP25"
}